skeletal muscle satellite cell maintenance involved in skeletal muscle regeneration [GO:0014834] (biological process) Relationships: is_a GO:0098727; is part of skeletal muscle tissue regeneration [GO:0043403] Definition: Any process by which the number of skeletal muscle satellite cells in a skeletal muscle is maintained during muscle regeneration. There are at least three mechanisms by which this is achieved. Skeletal muscle satellite stem cell asymmetric division ensures satellite stem cell numbers are kept constant. Symmetric division of these cells amplifies the number of skeletal muscle satellite stem cells. Some adult skeletal muscle myoblasts (descendants of activated satellite cells) can develop back into quiescent satellite cells, replenishing the overall pool of satellite cells. Subtypes: skeletal muscle satellite stem cell maintenance involved in skeletal muscle regeneration [GO:0098731] References: PMID:23303905 Sources: GOC:dph, GOC:ef, GOC:mtg_muscle, GOC:tb Also known as: satellite cell self-renewal, satellite cell compartment self-renewal involved in skeletal muscle regeneration, satellite cell population maintenance